{
  "gene_name": "Activating transcription factor 7-interacting protein 1",
  "term_id": "GO:0006355",
  "term_label": "regulation of DNA-templated transcription",
  "gene": "UniProtKB:Q6VMQ6",
  "gene_symbol": "ATF7IP"
}